oxidosqualene cyclase activity [GO:0031559] (molecular function) Subtypes: GO:0000250, cycloartenol synthase activity [GO:0016871], marneral synthase activity [GO:0034074], arabidiol synthase activity [GO:0034075], cucurbitadienol synthase activity [GO:0034076], GO:0042299, GO:0042300, alpha-amyrin synthase activity [GO:0042561], thalianol synthase activity [GO:0051746], GO:0080011 Sources: GOC:ct Note: Note that the phrase 'oxidosqualene cyclase' has been used to refer to enzymes that catalyze the reaction represented by 'lanosterol synthase activity ; GO:0000250'. Definition: Catalysis of the cyclization of (S)-2,3-epoxysqualene to form a triterpene. Relationships: is a type of intramolecular transferase activity [GO:0016866] Also known as: 2,3-oxidosqualene cyclase activity